positive regulation of pectin catabolic process [GO:2001005] (biological process) Also known as: positive regulation of pectin breakdown, positive regulation of pectin catabolism, positive regulation of pectin degradation Sources: GOC:mengo_curators Relationships: is a type of positive regulation of catabolic process [GO:0009896]; is a type of positive regulation of macromolecule metabolic process [GO:0010604]; is a type of positive regulation of carbohydrate metabolic process [GO:0045913]; is a type of regulation of pectin catabolic process [GO:2001003]; positively regulates pectin catabolic process [GO:0045490] Definition: Any process that activates or increases the frequency, rate or extent of pectin catabolic process.